positive regulation of epithelial to mesenchymal transition involved in endocardial cushion formation [GO:1905007] (biological process) Also known as: up regulation of epithelial to mesenchymal transition involved in endocardial cushion formation, up-regulation of epithelial to mesenchymal transition involved in endocardial cushion formation, upregulation of epithelial to mesenchymal transition involved in endocardial cushion formation, activation of epithelial to mesenchymal transition involved in endocardial cushion formation References: PMID:18718461 Sources: GOC:BHF, GOC:TermGenie, GOC:rl, GO_REF:0000058 Definition: Any process that activates or increases the frequency, rate or extent of epithelial to mesenchymal transition involved in endocardial cushion formation. Relationships: is a type of GO:0062043; is a type of regulation of epithelial to mesenchymal transition involved in endocardial cushion formation [GO:1905005]; positively regulates epithelial to mesenchymal transition involved in endocardial cushion formation [GO:0003198]